{
  "term_label": "glutamate-cysteine ligase complex",
  "gene_name": "Glutamate--cysteine ligase regulatory subunit",
  "term_id": "GO:0017109",
  "gene_symbol": "GCLM",
  "gene": "UniProtKB:P48507"
}